{
  "gene_symbol": "SEC31A",
  "term_id": "GO:0030127",
  "term_label": "COPII vesicle coat",
  "gene_name": "Protein transport protein Sec31A",
  "gene": "UniProtKB:O94979"
}